{
  "gene_name": "Hypermethylated in cancer 1 protein",
  "term_id": "GO:0005634",
  "gene": "UniProtKB:Q14526",
  "gene_symbol": "HIC1",
  "term_label": "nucleus"
}